{
  "gene": "UniProtKB:Q8NHC7",
  "gene_name": "Olfactory receptor 14C36",
  "gene_symbol": "OR14C36",
  "term_label": "olfactory receptor activity",
  "term_id": "GO:0004984"
}